{
  "gene_name": "5-hydroxytryptamine receptor 3C",
  "term_id": "GO:1904315",
  "gene": "UniProtKB:Q8WXA8",
  "gene_symbol": "HTR3C",
  "term_label": "transmitter-gated monoatomic ion channel activity involved in regulation of postsynaptic membrane potential"
}